L-arginine catabolic process to L-proline [GO:0019493] (biological process) Sources: GOC:go_curators Relationships: is a type of L-arginine catabolic process [GO:0006527]; is_a proline metabolic process [GO:0006560] Also known as: arginine breakdown to proline, arginine degradation to proline Subtypes: L-arginine catabolic process to proline via ornithine [GO:0010121] Definition: The chemical reactions and pathways resulting in the breakdown of L-arginine into other compounds, including L-proline.